{
  "term_id": "GO:0008021",
  "gene_name": "Neurotrophin-3",
  "term_label": "synaptic vesicle",
  "gene_symbol": "NTF3",
  "gene": "UniProtKB:P20783"
}